{
  "term_label": "CENP-A containing nucleosome",
  "gene_symbol": "CENPA",
  "gene": "UniProtKB:P49450",
  "term_id": "GO:0043505",
  "gene_name": "Histone H3-like centromeric protein A"
}